UDP-sugar diphosphatase activity [GO:0008768] (molecular function) Sources: EC:3.6.1.45 Relationships: is a type of pyrophosphatase activity [GO:0016462] Definition: Catalysis of the reaction: UDP-sugar + H2O = UMP + sugar 1-phosphate. Also known as: nucleosidediphosphate-sugar diphosphatase activity, nucleosidediphosphate-sugar pyrophosphatase activity, UDP-sugar hydrolase activity, UDP-sugar pyrophosphatase activity, UDP-sugar sugarphosphohydrolase activity